{
  "gene": "UniProtKB:Q86UW1",
  "gene_name": "Organic solute transporter subunit alpha",
  "term_id": "GO:0022857",
  "gene_symbol": "SLC51A",
  "term_label": "transmembrane transporter activity"
}